{
  "term_id": "GO:0071763",
  "gene_name": "Torsin-1B",
  "term_label": "nuclear membrane organization",
  "gene_symbol": "TOR1B",
  "gene": "UniProtKB:O14657"
}